{
  "gene_name": "Eukaryotic translation initiation factor 4E transporter",
  "gene_symbol": "EIF4ENIF1",
  "term_id": "GO:0017148",
  "gene": "UniProtKB:Q9NRA8",
  "term_label": "negative regulation of translation"
}